positive regulation of c-di-GMP signaling [GO:0061941] (biological process) Relationships: is a type of positive regulation of cell communication [GO:0010647]; is a type of positive regulation of signaling [GO:0023056]; is a type of regulation of c-di-GMP signaling [GO:0061940]; positively regulates c-di-GMP signaling [GO:0061939] Definition: Any process that increases the rate, frequency or extent of c-di-GMP signaling. References: PMID:22864416